regulation of postsynaptic specialization assembly [GO:0099150] (biological process) Relationships: is a type of GO:1902115; regulates postsynaptic specialization assembly [GO:0098698] Sources: GOC:dos Subtypes: regulation of postsynaptic density assembly [GO:0099151] Definition: Any process that modulates the frequency, rate or extent of postsynaptic specialization assembly, the aggregation, arrangement and bonding together of a set of components to form a postsynaptic specialization.